negative regulation of helvolic acid biosynthetic process [GO:1900841] (biological process) Sources: GOC:TermGenie, GOC:di Also known as: down regulation of helvolic acid biosynthetic process, down-regulation of helvolic acid biosynthetic process, downregulation of helvolic acid biosynthetic process Definition: Any process that stops, prevents or reduces the frequency, rate or extent of helvolic acid biosynthetic process. Relationships: is a type of negative regulation of steroid biosynthetic process [GO:0010894]; is a type of negative regulation of small molecule metabolic process [GO:0062014]; is a type of negative regulation of secondary metabolite biosynthetic process [GO:1900377]; is a type of GO:1900840; negatively regulates helvolic acid biosynthetic process [GO:1900812]